cocaine biosynthetic process [GO:0050799] (biological process) Definition: The chemical reactions and pathways resulting in the formation of cocaine, an alkaloid obtained from the dried leaves of the shrub Erythroxylon coca. It is a cerebral stimulant and narcotic. Sources: GOC:ai Relationships: is a type of tropane alkaloid biosynthetic process [GO:0009710] Also known as: cocaine anabolism, cocaine biosynthesis, cocaine formation, cocaine synthesis